olfactory nerve development [GO:0021553] (biological process) Sources: GOC:cls, GOC:dgh, GOC:dph, GOC:jid, GO_REF:0000021 Definition: The process whose specific outcome is the progression of the olfactory nerve over time, from its formation to the mature structure. The olfactory nerve is a collection of sensory nerve rootlets that extend down from the olfactory bulb to the olfactory mucosa of the upper parts of the nasal cavity. This nerve conducts odor information to the brainstem. Also known as: cranial nerve 1 development, cranial nerve I development, CN 1 development Relationships: is a type of GO:0021545